Wnt-protein binding [GO:0017147] (molecular function) Definition: Binding to a Wnt-protein, a secreted growth factor involved in signaling. Relationships: is_a protein binding [GO:0005515] Sources: GOC:jl